{
  "gene_symbol": "TMEM144",
  "gene_name": "Transmembrane protein 144",
  "gene": "UniProtKB:Q7Z5S9",
  "term_label": "Unknown biological process",
  "term_id": "UNKNOWN:0002"
}